{
  "term_id": "GO:0016567",
  "term_label": "protein ubiquitination",
  "gene": "UniProtKB:Q8IWV7",
  "gene_name": "E3 ubiquitin-protein ligase UBR1",
  "gene_symbol": "UBR1"
}